{
  "term_id": "UNKNOWN:0001",
  "gene_name": "Spindle and centriole-associated protein 1",
  "gene_symbol": "SPICE1",
  "term_label": "Unknown molecular function",
  "gene": "UniProtKB:Q8N0Z3"
}